{
  "gene_symbol": "ARHGAP17",
  "gene": "UniProtKB:Q68EM7",
  "term_label": "plasma membrane",
  "term_id": "GO:0005886",
  "gene_name": "Rho GTPase-activating protein 17"
}